{
  "gene": "UniProtKB:Q8WV37",
  "gene_name": "Zinc finger protein 480",
  "gene_symbol": "ZNF480",
  "term_label": "regulation of transcription by RNA polymerase II",
  "term_id": "GO:0006357"
}